{
  "term_id": "GO:0006233",
  "gene_name": "Thymidylate kinase",
  "term_label": "dTDP biosynthetic process",
  "gene_symbol": "DTYMK",
  "gene": "UniProtKB:P23919"
}